{
  "gene": "UniProtKB:P55769",
  "term_label": "small-subunit processome",
  "gene_name": "NHP2-like protein 1",
  "term_id": "GO:0032040",
  "gene_symbol": "SNU13"
}